{
  "gene_symbol": "CYP2R1",
  "term_id": "GO:0005737",
  "term_label": "cytoplasm",
  "gene": "UniProtKB:Q6VVX0",
  "gene_name": "Vitamin D 25-hydroxylase"
}